{
  "gene": "UniProtKB:A0A0J9YVY3",
  "gene_name": "Immunoglobulin heavy variable 7-4-1",
  "term_id": "GO:0003823",
  "term_label": "antigen binding",
  "gene_symbol": "IGHV7-4-1"
}